{
  "gene_name": "Glycosyl-phosphatidylinositol-anchored molecule-like protein",
  "gene": "UniProtKB:Q99445",
  "term_label": "Unknown molecular function",
  "gene_symbol": "GML",
  "term_id": "UNKNOWN:0001"
}